B cell homeostatic proliferation [GO:0002358] (biological process) Definition: The non-specific expansion of B cell populations within a whole or part of an organism to reach to a total number of B cells which will then remain stable over time in the absence of an external stimulus. Sources: GOC:jal Also known as: B lymphocyte homeostatic proliferation, B-cell homeostatic proliferation, B-lymphocyte homeostatic proliferation Relationships: is a type of GO:0042100; is part of homeostatic process [GO:0042592]